{
  "term_label": "negative regulation of DNA-templated transcription",
  "gene": "UniProtKB:Q8NB12",
  "gene_symbol": "SMYD1",
  "term_id": "GO:0045892",
  "gene_name": "Histone-lysine N-methyltransferase SMYD1"
}